{
  "gene": "UniProtKB:Q70CQ3",
  "gene_symbol": "USP30",
  "gene_name": "Ubiquitin carboxyl-terminal hydrolase 30",
  "term_label": "cytosol",
  "term_id": "GO:0005829"
}